osteoclast differentiation [GO:0030316] (biological process) Also known as: osteoclast cell differentiation Relationships: is a type of GO:0002573 Regulation: regulated by GO:0045670; negatively regulated by negative regulation of osteoclast differentiation [GO:0045671]; positively regulated by GO:0045672 Definition: The process in which a relatively unspecialized monocyte acquires the specialized features of an osteoclast. An osteoclast is a specialized phagocytic cell associated with the absorption and removal of the mineralized matrix of bone tissue. Subtypes: multinuclear osteoclast differentiation [GO:0072674] References: PMID:12161749 Sources: CL:0000092, GOC:add, ISBN:0781735149